glucuronate biosynthetic process [GO:0046399] (biological process) Subtypes: D-glucuronate biosynthetic process [GO:0042841] Also known as: glucuronate anabolism, glucuronate biosynthesis, glucuronate formation, glucuronate synthesis Relationships: is a type of glucuronate metabolic process [GO:0019585]; is a type of GO:0072330 Sources: GOC:ai Definition: The chemical reactions and pathways resulting in the formation of glucuronate, the anion of glucuronic acid.